{
  "gene": "UniProtKB:Q9BY19",
  "term_id": "GO:0005886",
  "gene_symbol": "MS4A8",
  "gene_name": "Membrane-spanning 4-domains subfamily A member 8",
  "term_label": "plasma membrane"
}